BRE1 E3 ubiquitin ligase complex [GO:1990352] (cellular component) Note: An example of this is BRE1 in Saccharomyces cerevisiae (UniProt symbol Q07457) in PMID:19531475 (inferred from direct assay). Definition: A homodimeric protein complex composed of the E3 ubiquitin-protein ligase BRE1. Plays a role in regulating association of RNA polymerase II with active genes. Relationships: is a type of ubiquitin ligase complex [GO:0000151] References: PMID:19531475 Sources: GOC:bhm Also known as: BRE1 E3 ubiquitin-protein ligase complex, BRE1 oligomer